{
  "term_id": "GO:0000813",
  "term_label": "ESCRT I complex",
  "gene": "UniProtKB:Q9H7P6",
  "gene_symbol": "MVB12B",
  "gene_name": "Multivesicular body subunit 12B"
}